{
  "term_label": "chromatin DNA binding",
  "gene_name": "TOX high mobility group box family member 3",
  "term_id": "GO:0031490",
  "gene_symbol": "TOX3",
  "gene": "UniProtKB:O15405"
}